{
  "gene_symbol": "UBA2",
  "term_label": "protein sumoylation",
  "gene_name": "SUMO-activating enzyme subunit 2",
  "term_id": "GO:0016925",
  "gene": "UniProtKB:Q9UBT2"
}